purine nucleotide-sugar transmembrane transporter activity [GO:0036080] (molecular function) Relationships: is a type of GO:0005338; is part of GO:0090480 References: PMID:19948734 Sources: GOC:sart Subtypes: GDP-fucose transmembrane transporter activity [GO:0005457], GDP-mannose transmembrane transporter activity [GO:0005458] Definition: Enables the transfer of a purine nucleotide-sugar from one side of a membrane to the other. Purine nucleotide-sugars are purine nucleotides in glycosidic linkage with a monosaccharide or monosaccharide derivative.